{
  "gene_symbol": "PIGC",
  "gene": "UniProtKB:Q92535",
  "gene_name": "Phosphatidylinositol N-acetylglucosaminyltransferase subunit C",
  "term_label": "Unknown molecular function",
  "term_id": "UNKNOWN:0001"
}